T-helper 17 cell extravasation [GO:0035699] (biological process) Sources: CL:0000899, GOC:BHF Relationships: is a type of helper T cell extravasation [GO:0035684]; is a type of CD8-positive, alpha-beta T cell extravasation [GO:0035697] Definition: The migration of a T-helper 17 cell from the blood vessels into the surrounding tissue. Regulation: regulated by regulation of T-helper 17 cell extravasation [GO:2000455]; negatively regulated by negative regulation of T-helper 17 cell extravasation [GO:2000456]; positively regulated by positive regulation of T-helper 17 cell extravasation [GO:2000457]